{
  "gene_symbol": "KIF20B",
  "term_label": "microtubule-based movement",
  "term_id": "GO:0007018",
  "gene": "UniProtKB:Q96Q89",
  "gene_name": "Kinesin-like protein KIF20B"
}